glucose-1-phosphate adenylyltransferase activity [GO:0008878] (molecular function) Also known as: ADGase activity, ADPG pyrophosphorylase activity, ATP:alpha-glucose-1-phosphate adenylyl transferase activity, ADP glucose pyrophosphorylase activity, ADP-glucose diphosphorylase activity, ADP-glucose pyrophosphorylase activity, ADP-glucose synthase activity, ADP-glucose synthetase activity, ADP:alpha-D-glucose-1-phosphate adenylyltransferase activity, ATP:alpha-D-glucose-1-phosphate adenylyltransferase activity, adenosine diphosphate glucose pyrophosphorylase activity, adenosine diphosphoglucose pyrophosphorylase activity, glucose 1-phosphate adenylyltransferase activity Sources: EC:2.7.7.27, RHEA:12120 Relationships: is a type of adenylyltransferase activity [GO:0070566] Definition: Catalysis of the reaction: alpha-D-glucose 1-phosphate + ATP = ADP-glucose + diphosphate.